regulation of adaptive immune response based on somatic recombination of immune receptors built from immunoglobulin superfamily domains [GO:0002822] (biological process) Relationships: is a type of regulation of adaptive immune response [GO:0002819]; regulates GO:0002460 Subtypes: regulation of germinal center formation [GO:0002634], regulation of tolerance induction dependent upon immune response [GO:0002652], regulation of T cell mediated immunity [GO:0002709], GO:0002712, negative regulation of adaptive immune response based on somatic recombination of immune receptors built from immunoglobulin superfamily domains [GO:0002823], positive regulation of adaptive immune response based on somatic recombination of immune receptors built from immunoglobulin superfamily domains [GO:0002824], regulation of T-helper 1 type immune response [GO:0002825], regulation of T-helper 17 type immune response [GO:2000316] Sources: GOC:add, GOC:mtg_sensu Definition: Any process that modulates the frequency, rate, or extent of an adaptive immune response based on somatic recombination of immune receptors built from immunoglobulin superfamily domains. An example of this process is found in the Gnathostomata.